{
  "gene": "UniProtKB:P17039",
  "gene_symbol": "ZNF30",
  "term_id": "GO:0000978",
  "term_label": "RNA polymerase II cis-regulatory region sequence-specific DNA binding",
  "gene_name": "Zinc finger protein 30"
}